central B cell receptor editing [GO:0002511] (biological process) Definition: Receptor editing occurring in B cells in the bone marrow. References: PMID:16460922 Sources: GOC:jal Also known as: central B lymphocyte receptor editing, central B-cell receptor editing, central B-lymphocyte receptor editing Relationships: is a type of B cell receptor editing [GO:0002452]